{
  "gene_symbol": "KCTD11",
  "gene_name": "BTB_POZ domain-containing protein KCTD11",
  "term_id": "GO:0045666",
  "term_label": "positive regulation of neuron differentiation",
  "gene": "UniProtKB:Q693B1"
}